{
  "gene_name": "Olfactory receptor 8K5",
  "term_id": "UNKNOWN:0003",
  "gene_symbol": "OR8K5",
  "term_label": "Unknown cellular component",
  "gene": "UniProtKB:Q8NH50"
}